{
  "term_id": "GO:0005737",
  "gene_name": "Tubulin alpha-3D chain",
  "gene_symbol": "TUBA3D",
  "term_label": "cytoplasm",
  "gene": "UniProtKB:P0DPH8"
}